{
  "gene": "UniProtKB:Q6ZWB6",
  "gene_symbol": "KCTD8",
  "gene_name": "BTB_POZ domain-containing protein KCTD8",
  "term_id": "GO:0043235",
  "term_label": "receptor complex"
}